folic acid:proton symporter activity [GO:0140211] (molecular function) References: PMID:24745983 Definition: Enables the transfer of a solute or solutes from one side of a membrane to the other according to the reaction: folic acid(out) + H+(out) = folic acid(in) + H+(in). The main folic acid symporter is the Proton-Coupled Folate Transporter (PCFT/SLC46A1), which has similar affinity for transport of reduced folates (5-methyl THF, 5-formyl THF) and folic acid. Relationships: is a type of folic acid transmembrane transporter activity [GO:0008517]; is a type of solute:proton symporter activity [GO:0015295]